{
  "gene": "UniProtKB:A0A1W2PQU2",
  "gene_name": "KANTR integral membrane protein",
  "term_label": "Unknown molecular function",
  "gene_symbol": "KANTR",
  "term_id": "UNKNOWN:0001"
}